{
  "gene": "UniProtKB:Q8N339",
  "term_id": "GO:0046872",
  "gene_symbol": "MT1M",
  "term_label": "metal ion binding",
  "gene_name": "Metallothionein-1M"
}